{
  "term_id": "UNKNOWN:0003",
  "gene_name": "Putative uncharacterized protein FLJ46214",
  "gene": "UniProtKB:Q6ZRN7",
  "gene_symbol": "Q6ZRN7",
  "term_label": "Unknown cellular component"
}